{
  "term_label": "RNA polymerase II complex binding",
  "gene_name": "RNA polymerase II-associated factor 1 homolog",
  "term_id": "GO:0000993",
  "gene_symbol": "PAF1",
  "gene": "UniProtKB:Q8N7H5"
}